costunolide synthase activity [GO:0102934] (molecular function) Sources: GOC:pz, RHEA:28230 Definition: Catalysis of the reaction: germacra-1(10),4,11(13)-trien-12-oate + O2 + NADPH + 2 H+ = costunolide + 2 H2O + NADP. Relationships: is a type of oxidoreductase activity, acting on paired donors, with incorporation or reduction of molecular oxygen, NAD(P)H as one donor, and incorporation of one atom of oxygen [GO:0016709]